{
  "term_id": "GO:0005654",
  "gene_name": "G-rich sequence factor 1",
  "gene_symbol": "GRSF1",
  "term_label": "nucleoplasm",
  "gene": "UniProtKB:Q12849"
}